O-demethylpuromycin O-methyltransferase activity [GO:0030739] (molecular function) Definition: Catalysis of the reaction: S-adenosyl-L-methionine + O-demethylpuromycin = S-adenosyl-L-homocysteine + puromycin. Also known as: O-demethylpuromycin methyltransferase activity, S-adenosyl-L-methionine:O-demethylpuromycin O-methyltransferase activity Sources: EC:2.1.1.38 Relationships: is a type of S-adenosylmethionine-dependent methyltransferase activity [GO:0008757]